{
  "gene_name": "DNA-directed RNA polymerase III subunit RPC9",
  "gene_symbol": "CRCP",
  "term_id": "UNKNOWN:0001",
  "gene": "UniProtKB:O75575",
  "term_label": "Unknown molecular function"
}